STING complex [GO:1990231] (cellular component) Definition: A protein dimer containing two STING monomers. It binds cyclic purine di-nucleotides. Activation of the sting complex by 2',5'-3'-5'-cyclic GMP-AMP activates nuclear transcription factor kB (NF-kB) and interferon regulatory factor 3 (IRF3) which then induce transcription of the genes encoding type I IFN and cytokines active in the innate immune response. Relationships: is a type of membrane protein complex [GO:0098796]; is part of cytoplasmic vesicle membrane [GO:0030659] Also known as: stimulator of interferon genes complex References: PMID:22705373, PMID:23706668, PMID:23910378 Sources: GOC:bhm